{
  "gene_name": "Low-density lipoprotein receptor class A domain-containing protein 4",
  "term_label": "Golgi membrane",
  "term_id": "GO:0000139",
  "gene": "UniProtKB:O15165",
  "gene_symbol": "LDLRAD4"
}